{
  "gene": "UniProtKB:P53567",
  "gene_name": "CCAAT_enhancer-binding protein gamma",
  "term_label": "DNA-binding transcription factor activity, RNA polymerase II-specific",
  "term_id": "GO:0000981",
  "gene_symbol": "CEBPG"
}